L-lysine 4-chlorinase activity [GO:0062147] (molecular function) Definition: Catalysis of the reaction: 2-oxoglutarate + chloride + H+ + L-lysine + O2 = 4-chloro-L-lysine + CO2 + H2O + succinate. Relationships: is a type of GO:0050498 References: PMID:30867596 Sources: RHEA:59884